{
  "term_id": "GO:0098632",
  "gene_symbol": "NTNG2",
  "term_label": "cell-cell adhesion mediator activity",
  "gene_name": "Netrin-G2",
  "gene": "UniProtKB:Q96CW9"
}